{
  "gene_name": "Transcriptional repressor NF-X1",
  "term_label": "nucleus",
  "gene": "UniProtKB:Q12986",
  "gene_symbol": "NFX1",
  "term_id": "GO:0005634"
}